{
  "term_label": "ATP hydrolysis activity",
  "term_id": "GO:0016887",
  "gene_name": "Putative heat shock protein HSP 90-beta 4",
  "gene": "UniProtKB:Q58FF6",
  "gene_symbol": "HSP90AB4P"
}